{
  "gene_name": "Potassium_sodium hyperpolarization-activated cyclic nucleotide-gated channel 3",
  "gene_symbol": "HCN3",
  "term_id": "GO:0005249",
  "gene": "UniProtKB:Q9P1Z3",
  "term_label": "voltage-gated potassium channel activity"
}